histone H1K75 acetyltransferase activity [GO:0160263] (MF) Relationships: is_a histone H1 acetyltransferase activity [GO:0160262] Definition: Catalysis of the reaction: acetyl-CoA + histone H1 L-lysine (position 75) = CoA + histone H1 N6-acetyl-L-lysine (position 75). References: PMID:40240600